{
  "term_id": "GO:0032481",
  "gene_symbol": "IKBKE",
  "gene": "UniProtKB:Q14164",
  "term_label": "positive regulation of type I interferon production",
  "gene_name": "Inhibitor of nuclear factor kappa-B kinase subunit epsilon"
}